{
  "gene_symbol": "TRPC5",
  "term_label": "calcium ion transmembrane transport",
  "gene_name": "Short transient receptor potential channel 5",
  "gene": "UniProtKB:Q9UL62",
  "term_id": "GO:0070588"
}